{
  "gene": "UniProtKB:Q30201",
  "gene_symbol": "HFE",
  "gene_name": "Hereditary hemochromatosis protein",
  "term_label": "extracellular space",
  "term_id": "GO:0005615"
}